{
  "gene_name": "Zinc finger protein 397",
  "term_label": "Unknown cellular component",
  "term_id": "UNKNOWN:0003",
  "gene": "UniProtKB:Q8NF99",
  "gene_symbol": "ZNF397"
}